{
  "gene_name": "Transducin-like enhancer protein 4",
  "term_id": "GO:0090090",
  "term_label": "negative regulation of canonical Wnt signaling pathway",
  "gene_symbol": "TLE4",
  "gene": "UniProtKB:Q04727"
}